{
  "term_id": "GO:0005737",
  "gene_symbol": "SLK",
  "term_label": "cytoplasm",
  "gene_name": "STE20-like serine_threonine-protein kinase",
  "gene": "UniProtKB:Q9H2G2"
}